rRNA pseudouridine synthesis [GO:0031118] (biological process) Sources: GOC:mah Relationships: is a type of rRNA modification [GO:0000154]; is a type of pseudouridine synthesis [GO:0001522] Subtypes: snoRNA guided rRNA pseudouridine synthesis [GO:0000454], GO:0000455 Definition: The intramolecular conversion of uridine to pseudouridine in an rRNA molecule.